{
  "gene": "UniProtKB:P62952",
  "gene_name": "Bladder cancer-associated protein",
  "term_label": "Unknown biological process",
  "term_id": "UNKNOWN:0002",
  "gene_symbol": "BLCAP"
}